protein import into mitochondrial intermembrane space [GO:0045041] (biological process) Also known as: mitochondrial intermembrane space protein import, protein import into mitochondrial IMS, protein transport into mitochondrial IMS, protein transport into mitochondrial intermembrane space, protein import into mitochondrial intermembrane space, direct, protein import into mitochondrial intermembrane space, nonconservative Relationships: is a type of protein localization to mitochondrion [GO:0070585]; is a type of protein transmembrane transport [GO:0071806]; is a type of establishment of protein localization to mitochondrion [GO:0072655] Definition: The import of proteins into the space between the inner and outer mitochondrial membranes. Sources: ISBN:0716731363